{
  "term_label": "immunoglobulin mediated immune response",
  "gene_symbol": "IGHV3-11",
  "gene_name": "Immunoglobulin heavy variable 3-11",
  "gene": "UniProtKB:P01762",
  "term_id": "GO:0016064"
}